membrane potential driven uniporter activity [GO:0022810] (MF) Relationships: is a type of uniporter activity [GO:0015292] Definition: Enables the active transport of a solute across a membrane by a mechanism involving conformational change, where energy for active transport is derived from membrane potential if the solute is charged. Subtypes: sodium ion uniporter activity [GO:0022818], potassium ion uniporter activity [GO:0022819], GO:0140787, L-glutamate uniporter activity [GO:0140788], GO:0160042 Sources: GOC:mtg_transport, ISBN:0815340729 Also known as: porter